{
  "gene_name": "Tyrosine 3-monooxygenase",
  "term_id": "GO:0004511",
  "term_label": "tyrosine 3-monooxygenase activity",
  "gene_symbol": "TH",
  "gene": "UniProtKB:P07101"
}